{
  "term_label": "Unknown molecular function",
  "gene_symbol": "TMEM179B",
  "term_id": "UNKNOWN:0001",
  "gene": "UniProtKB:Q7Z7N9",
  "gene_name": "Transmembrane protein 179B"
}